{
  "gene_symbol": "IFT20",
  "term_label": "cilium assembly",
  "term_id": "GO:0060271",
  "gene_name": "Intraflagellar transport protein 20 homolog",
  "gene": "UniProtKB:Q8IY31"
}